has_narrow_synonym [oboInOwl#hasNarrowSynonym]